{
  "term_id": "GO:0005737",
  "gene": "UniProtKB:Q8N752",
  "gene_symbol": "CSNK1A1L",
  "term_label": "cytoplasm",
  "gene_name": "Casein kinase I isoform alpha-like"
}